{
  "term_label": "immune system development",
  "gene_symbol": "GATA3",
  "gene": "UniProtKB:P23771",
  "term_id": "GO:0002520",
  "gene_name": "Trans-acting T-cell-specific transcription factor GATA-3"
}